{
  "gene_name": "Secreted and transmembrane protein 1",
  "gene_symbol": "SECTM1",
  "term_label": "Unknown molecular function",
  "term_id": "UNKNOWN:0001",
  "gene": "UniProtKB:Q8WVN6"
}